{
  "gene_symbol": "SLC7A9",
  "term_label": "L-cystine transmembrane transporter activity",
  "gene_name": "b(0,+)-type amino acid transporter 1",
  "term_id": "GO:0015184",
  "gene": "UniProtKB:P82251"
}